{
  "gene": "UniProtKB:Q0P5N6",
  "term_label": "Unknown cellular component",
  "gene_symbol": "ARL16",
  "term_id": "UNKNOWN:0003",
  "gene_name": "ADP-ribosylation factor-like protein 16"
}